{
  "term_label": "DNA binding",
  "gene_name": "Tigger transposable element-derived protein 1",
  "term_id": "GO:0003677",
  "gene": "UniProtKB:Q96MW7",
  "gene_symbol": "TIGD1"
}